{
  "gene_symbol": "SLC30A8",
  "gene": "UniProtKB:Q8IWU4",
  "gene_name": "Proton-coupled zinc antiporter SLC30A8",
  "term_label": "zinc ion transmembrane transporter activity",
  "term_id": "GO:0005385"
}